{
  "term_label": "mitochondrion",
  "gene": "UniProtKB:Q8N4E7",
  "gene_symbol": "FTMT",
  "gene_name": "Ferritin, mitochondrial",
  "term_id": "GO:0005739"
}